{
  "gene_name": "Oxidized low-density lipoprotein receptor 1",
  "term_id": "GO:0007159",
  "term_label": "leukocyte cell-cell adhesion",
  "gene_symbol": "OLR1",
  "gene": "UniProtKB:P78380"
}